regulation of oxidoreductase activity [GO:0051341] (biological process) Relationships: is a type of GO:0050790; regulates oxidoreductase activity [GO:0016491] Definition: Any process that modulates the frequency, rate or extent of oxidoreductase activity, the catalysis of an oxidation-reduction (redox) reaction, a reversible chemical reaction in which the oxidation state of an atom or atoms within a molecule is altered. One substrate acts as a hydrogen or electron donor and becomes oxidized, while the other acts as hydrogen or electron acceptor and becomes reduced. Also known as: oxidoreductase regulator Subtypes: regulation of nitric-oxide synthase activity [GO:0050999], GO:0051353, negative regulation of oxidoreductase activity [GO:0051354], regulation of superoxide dismutase activity [GO:1901668] Sources: GOC:ai